{
  "term_label": "DNA-binding transcription factor activity, RNA polymerase II-specific",
  "gene_symbol": "SP5",
  "gene": "UniProtKB:Q6BEB4",
  "gene_name": "Transcription factor Sp5",
  "term_id": "GO:0000981"
}